NK T cell proliferation involved in immune response [GO:0002289] (biological process) Also known as: NK T cell proliferation during immune response, NK T lymphocyte proliferation during immune response, NK T-cell proliferation during immune response, NK T-lymphocyte proliferation during immune response, natural killer T lymphocyte proliferation during immune response, natural killer T-cell proliferation during immune response, natural killer T-lymphocyte proliferation during immune response Relationships: is_a NK T cell proliferation [GO:0001866]; is_a NK T cell activation involved in immune response [GO:0002288]; is_a alpha-beta T cell proliferation involved in immune response [GO:0002310] References: PMID:15771592 Sources: GOC:add Definition: The expansion of a NK T cell population by cell division as part of an immune response.